{
  "gene_symbol": "SCAMP3",
  "term_id": "GO:0032588",
  "gene_name": "Secretory carrier-associated membrane protein 3",
  "term_label": "trans-Golgi network membrane",
  "gene": "UniProtKB:O14828"
}